regulation of leukocyte apoptotic process [GO:2000106] (biological process) Also known as: regulation of leukocyte apoptosis Definition: Any process that modulates the frequency, rate or extent of leukocyte apoptotic process. Sources: GOC:BHF, GOC:mtg_apoptosis Relationships: is_a regulation of apoptotic process [GO:0042981]; RO_0002211 leukocyte apoptotic process [GO:0071887] Subtypes: regulation of mast cell apoptotic process [GO:0033025], regulation of neutrophil apoptotic process [GO:0033029], GO:0070228, negative regulation of leukocyte apoptotic process [GO:2000107], positive regulation of leukocyte apoptotic process [GO:2000108], GO:2000109, GO:2000668